{
  "gene": "UniProtKB:Q8IWE2",
  "term_label": "Unknown molecular function",
  "gene_name": "Protein NOXP20",
  "term_id": "UNKNOWN:0001",
  "gene_symbol": "FAM114A1"
}